{
  "gene": "UniProtKB:Q8TE54",
  "gene_symbol": "SLC26A7",
  "gene_name": "Anion exchange transporter",
  "term_label": "sulfate transmembrane transport",
  "term_id": "GO:1902358"
}